{
  "gene": "UniProtKB:P81408",
  "gene_name": "Protein ENTREP3",
  "gene_symbol": "ENTREP3",
  "term_label": "Unknown cellular component",
  "term_id": "UNKNOWN:0003"
}